ATPase-coupled urea transmembrane transporter activity [GO:0033221] (molecular function) Sources: GOC:mlg Relationships: is a type of urea transmembrane transporter activity [GO:0015204]; is a type of ATPase-coupled transmembrane transporter activity [GO:0042626] Definition: Catalysis of the reaction: ATP + H2O + urea(out) = ADP + phosphate + urea(in). Also known as: ATP-dependent urea transmembrane transporter activity, carbamide-transporting ATPase activity, urea-transporting ATPase activity